mesonephric interstitial fibroblast fate commitment [GO:0061268] (biological process) Relationships: is a type of renal interstitial fibroblast fate commitment [GO:0072153]; is part of mesonephric interstitial fibroblast differentiation [GO:0061266] Sources: GOC:mtg_kidney_jan10 Definition: The process in which the developmental fate of a cell becomes restricted such that it will develop into a mesonephric interstitial fibroblast.